{
  "term_id": "GO:0003729",
  "gene_symbol": "SLC4A1AP",
  "term_label": "mRNA binding",
  "gene_name": "Kanadaptin",
  "gene": "UniProtKB:Q9BWU0"
}